{
  "gene": "UniProtKB:P55290",
  "gene_name": "Cadherin-13",
  "gene_symbol": "CDH13",
  "term_id": "GO:0008013",
  "term_label": "beta-catenin binding"
}